positive regulation of wound healing [GO:0090303] (biological process) Definition: Any process that increases the rate, frequency, or extent of the series of events that restore integrity to a damaged tissue, following an injury. Subtypes: positive regulation of blood coagulation [GO:0030194], positive regulation of vascular wound healing [GO:0035470], positive regulation of wound healing, spreading of epidermal cells [GO:1903691] Relationships: is a type of regulation of wound healing [GO:0061041]; is_a positive regulation of response to wounding [GO:1903036]; positively regulates wound healing [GO:0042060] Sources: GOC:BHF